{
  "gene": "UniProtKB:Q30KR1",
  "term_id": "GO:0042742",
  "gene_symbol": "DEFB109B",
  "term_label": "defense response to bacterium",
  "gene_name": "Putative beta-defensin 109B"
}